{
  "gene": "UniProtKB:A0A075B6Z3",
  "gene_symbol": "TRAJ6",
  "term_id": "UNKNOWN:0003",
  "term_label": "Unknown cellular component",
  "gene_name": "T cell receptor alpha joining 6 (Fragment)"
}